{
  "gene_name": "Uncharacterized protein C5orf64",
  "gene_symbol": "C5orf64",
  "gene": "UniProtKB:Q2M2E5",
  "term_id": "UNKNOWN:0001",
  "term_label": "Unknown molecular function"
}